{
  "gene_symbol": "PIP5K1C",
  "gene": "UniProtKB:O60331",
  "term_id": "GO:0016308",
  "gene_name": "Phosphatidylinositol 4-phosphate 5-kinase type-1 gamma",
  "term_label": "1-phosphatidylinositol-4-phosphate 5-kinase activity"
}